{
  "term_id": "GO:0015810",
  "gene": "UniProtKB:Q6NSJ5",
  "gene_symbol": "LRRC8E",
  "gene_name": "Volume-regulated anion channel subunit LRRC8E",
  "term_label": "aspartate transmembrane transport"
}